Golgi stack [GO:0005795] (cellular component) Definition: The set of thin, flattened membrane-bounded compartments, called cisternae, that form the central portion of the Golgi complex. The stack usually comprises cis, medial, and trans cisternae; the cis- and trans-Golgi networks are not considered part of the stack. Sources: GOC:mah, ISBN:0815316194 Relationships: is a type of Golgi apparatus subcompartment [GO:0098791] Also known as: Golgi cisternae, dictyosome